{
  "term_label": "pattern recognition receptor activity",
  "gene": "UniProtKB:P06734",
  "gene_symbol": "FCER2",
  "term_id": "GO:0038187",
  "gene_name": "Low affinity immunoglobulin epsilon Fc receptor"
}